{
  "gene": "UniProtKB:P35638",
  "gene_symbol": "DDIT3",
  "term_id": "GO:1990617",
  "gene_name": "DNA damage-inducible transcript 3 protein",
  "term_label": "CHOP-ATF4 complex"
}